{
  "gene": "UniProtKB:O43921",
  "term_label": "bone remodeling",
  "gene_symbol": "EFNA2",
  "gene_name": "Ephrin-A2",
  "term_id": "GO:0046849"
}